{
  "gene_name": "Immunoglobulin heavy diversity 3-3 (Fragment)",
  "gene_symbol": "IGHD3-3",
  "term_label": "Unknown biological process",
  "gene": "UniProtKB:A0A0J9YWD0",
  "term_id": "UNKNOWN:0002"
}